cellular response to glucose starvation [GO:0042149] (biological process) Relationships: is a type of GO:0009267 Definition: Any process that results in a change in state or activity of a cell (in terms of movement, secretion, enzyme production, gene expression, etc.) as a result of deprivation of glucose. Sources: GOC:jl Regulation: regulated by regulation of cellular response to glucose starvation [GO:1904547] Subtypes: positive regulation of protein export from nucleus in response to glucose starvation [GO:0036279]